{
  "gene": "UniProtKB:Q96PC5",
  "term_label": "endoplasmic reticulum to Golgi vesicle-mediated transport",
  "gene_symbol": "MIA2",
  "gene_name": "Melanoma inhibitory activity protein 2",
  "term_id": "GO:0006888"
}